somatostatin signaling pathway [GO:0038170] (biological process) Also known as: SRIF signaling pathway, SST signaling pathway, somatostatin signalling pathway, somatostatin-activated somatostatin receptor signaling pathway, somatostatin-mediated signaling pathway, somatotrophin release inhibiting factor signaling pathway References: PMID:18006219 Sources: GOC:bf, GOC:nhn, GOC:signaling, Wikipedia:Somatostatin Relationships: is_a hormone-mediated signaling pathway [GO:0009755]; is_a somatostatin receptor signaling pathway [GO:0038169] Definition: A G protein-coupled receptor signaling pathway initiated by somatostatin binding to a somatostatin receptor (SSTR), and ending with the regulation of a downstream cellular process, e.g. transcription.